{
  "gene": "UniProtKB:P41597",
  "term_label": "calcium-mediated signaling",
  "gene_name": "C-C chemokine receptor type 2",
  "gene_symbol": "CCR2",
  "term_id": "GO:0019722"
}